diamine N-acetyltransferase activity [GO:0004145] (molecular function) Sources: RHEA:11116 Definition: Catalysis of the reaction: an alkane-alpha,omega-diamine + acetyl-CoA = an N-acetylalkane-alpha,omega-diamine + CoA + H+. Relationships: is a type of N-acetyltransferase activity [GO:0008080] Also known as: diamine acetyltransferase activity, acetyl-coenzyme A-1,4-diaminobutane N-acetyltransferase activity, putrescine (diamine)-acetylating enzyme activity, putrescine N-acetyltransferase activity, putrescine acetylase activity, putrescine acetyltransferase activity, spermidine N(1)-acetyltransferase activity, spermidine acetyltransferase activity, spermine N(1)-acetyltransferase, spermine acetyltransferase, acetyl-CoA:alkane-alpha,omega-diamine N-acetyltransferase activity, spermidine N1-acetyltransferase activity, spermidine/spermine N1-acetyltransferase activity, spermine N-acetyltransferase